{
  "gene_symbol": "PRR20D",
  "term_id": "UNKNOWN:0003",
  "term_label": "Unknown cellular component",
  "gene_name": "Proline-rich protein 20D",
  "gene": "UniProtKB:P86480"
}